{
  "term_id": "GO:0032099",
  "gene": "UniProtKB:Q99988",
  "gene_name": "Growth_differentiation factor 15",
  "term_label": "negative regulation of appetite",
  "gene_symbol": "GDF15"
}